histone H3K27 acetyltransferase activity [GO:0044017] (molecular function) Relationships: is a type of histone H3 acetyltransferase activity [GO:0010484] Definition: Catalysis of the reaction: acetyl-CoA + histone H3 L-lysine (position 27) = CoA + histone H3 N6-acetyl-L-lysine (position 27). Note: Comment: Note that the residue position corresponds to the canonical human H3 histone (UniProtKB:P84243); this residue is conserved across all eukaryotes. Residue 1 is the first residue following removal of the initiating Methionine (Met). Note that each histone is encoded by multiple genes, and sequences may vary across different genes within an organism. References: PMID:18552846 Also known as: histone H3-K27 acetyltransferase activity, histone acetylase activity (H3-K27 specific), histone acetyltransferase activity (H3-K27 specific), histone lysine N-acetyltransferase activity (H3-K27 specific)